{
  "term_label": "endoplasmic reticulum to Golgi vesicle-mediated transport",
  "term_id": "GO:0006888",
  "gene": "UniProtKB:Q13445",
  "gene_name": "Transmembrane emp24 domain-containing protein 1",
  "gene_symbol": "TMED1"
}